{
  "gene_symbol": "CHPT1",
  "term_id": "UNKNOWN:0002",
  "gene_name": "Cholinephosphotransferase 1",
  "term_label": "Unknown biological process",
  "gene": "UniProtKB:Q8WUD6"
}